metanephric podocyte development [GO:0072249] (biological process) Sources: GOC:mtg_kidney_jan10 Relationships: is a type of GO:0072015; is a type of metanephric glomerular epithelial cell development [GO:0072313]; is part of metanephric podocyte differentiation [GO:0072248] Definition: The process whose specific outcome is the progression of a metanephric glomerular visceral epithelial cell over time, from its formation to the mature structure. A metanephric glomerular visceral epithelial cell is a specialized epithelial cell that contains 'feet' that interdigitate with the 'feet' of other glomerular epithelial cells in the metanephros. Regulation: regulated by GO:2000477; positively regulated by GO:2000478 Also known as: metanephric glomerular visceral epithelial cell development